{
  "term_id": "GO:0046470",
  "term_label": "phosphatidylcholine metabolic process",
  "gene": "UniProtKB:Q9NZK7",
  "gene_name": "Group IIE secretory phospholipase A2",
  "gene_symbol": "PLA2G2E"
}